{
  "term_id": "GO:0005886",
  "gene": "UniProtKB:Q96P88",
  "gene_symbol": "GNRHR2",
  "term_label": "plasma membrane",
  "gene_name": "Putative gonadotropin-releasing hormone II receptor"
}